IDP phosphatase activity [GO:1990003] (molecular function) Relationships: is a type of nucleoside diphosphate phosphatase activity [GO:0017110] References: PMID:20385596, PMID:22849572 Sources: RHEA:35207 Definition: Catalysis of the reaction: IDP + H2O = IMP + H+ + phosphate. Also known as: IDP diphosphatase activity, IDPase activity, inosine diphosphatase activity, inosine-diphosphatase activity